{
  "gene": "UniProtKB:Q9P0P8",
  "term_id": "GO:1903108",
  "gene_symbol": "MTRES1",
  "gene_name": "Mitochondrial transcription rescue factor 1",
  "term_label": "regulation of mitochondrial transcription"
}